{
  "gene": "UniProtKB:Q86SF2",
  "term_label": "polypeptide N-acetylgalactosaminyltransferase activity",
  "term_id": "GO:0004653",
  "gene_name": "N-acetylgalactosaminyltransferase 7",
  "gene_symbol": "GALNT7"
}